Enterobacter ribonuclease activity [GO:0008847] (MF) Definition: Catalysis of the endonucleolytic cleavage to 3'-phosphomononucleotides and 3'-phosphooligonucleotides with 2',3'-cyclic phosphate intermediates. Sources: EC:4.6.1.21 Also known as: Enterobacter RNase activity Relationships: is a type of RNA endonuclease activity [GO:0004521]; is a type of phosphorus-oxygen lyase activity [GO:0016849]